{
  "gene": "UniProtKB:A6NN90",
  "gene_symbol": "C2orf81",
  "term_id": "UNKNOWN:0002",
  "gene_name": "Uncharacterized protein C2orf81",
  "term_label": "Unknown biological process"
}